{
  "term_id": "GO:0061631",
  "gene": "UniProtKB:P63146",
  "term_label": "ubiquitin conjugating enzyme activity",
  "gene_name": "Ubiquitin-conjugating enzyme E2 B",
  "gene_symbol": "UBE2B"
}